{
  "gene_symbol": "ARHGAP42",
  "gene_name": "Rho GTPase-activating protein 42",
  "gene": "UniProtKB:A6NI28",
  "term_label": "GTPase activator activity",
  "term_id": "GO:0005096"
}